{
  "term_id": "GO:1903278",
  "gene_symbol": "FXYD1",
  "gene_name": "Phospholemman",
  "gene": "UniProtKB:O00168",
  "term_label": "positive regulation of sodium ion export across plasma membrane"
}